{
  "term_label": "plasma membrane",
  "gene": "UniProtKB:Q16651",
  "term_id": "GO:0005886",
  "gene_name": "Prostasin",
  "gene_symbol": "PRSS8"
}